chenodeoxycholoyltaurine hydrolase activity [GO:0047742] (molecular function) Relationships: is a type of hydrolase activity, acting on carbon-nitrogen (but not peptide) bonds, in linear amides [GO:0016811] Also known as: chenodeoxycholoyltaurine amidohydrolase activity Definition: Catalysis of the reaction: chenodeoxycholoyltaurine + H2O = chenodeoxycholate + taurine. Sources: EC:3.5.1.74, MetaCyc:CHENODEOXYCHOLOYLTAURINE-HYDROLASE-RXN